tricuspid valve formation [GO:0003195] (biological process) Definition: The developmental process pertaining to the initial formation of the tricuspid valve from unspecified parts. This process begins with the specific processes that contribute to the appearance of the discrete structure and ends when the structural rudiment is recognizable. Sources: GOC:mtg_heart Relationships: is a type of atrioventricular valve formation [GO:0003190]; is part of tricuspid valve morphogenesis [GO:0003186]